{
  "term_label": "cellular response to leucine starvation",
  "gene": "UniProtKB:P58005",
  "gene_name": "Sestrin-3",
  "term_id": "GO:1990253",
  "gene_symbol": "SESN3"
}